{
  "term_id": "GO:0005634",
  "gene_symbol": "IRX5",
  "term_label": "nucleus",
  "gene_name": "Iroquois-class homeodomain protein IRX-5",
  "gene": "UniProtKB:P78411"
}